{
  "gene": "UniProtKB:P32321",
  "gene_name": "Deoxycytidylate deaminase",
  "term_id": "GO:0006231",
  "gene_symbol": "DCTD",
  "term_label": "dTMP biosynthetic process"
}